{
  "term_label": "regulation of transcription by RNA polymerase II",
  "gene_symbol": "FOXK2",
  "gene_name": "Forkhead box protein K2",
  "term_id": "GO:0006357",
  "gene": "UniProtKB:Q01167"
}